{
  "gene_name": "Cytochrome P450 4V2",
  "term_label": "Unknown molecular function",
  "gene": "UniProtKB:Q6ZWL3",
  "gene_symbol": "CYP4V2",
  "term_id": "UNKNOWN:0001"
}